fluoride transmembrane transport [GO:1903424] (biological process) Subtypes: GO:0140116 Definition: The process in which fluoride is transported across a membrane. Relationships: is a type of GO:0015698; is a type of monoatomic anion transmembrane transport [GO:0098656] Also known as: fluoride membrane transport, transmembrane fluoride transport References: PMID:24173035 Sources: GOC:TermGenie, GO_REF:0000069